{
  "gene": "UniProtKB:Q9Y255",
  "term_id": "UNKNOWN:0001",
  "term_label": "Unknown molecular function",
  "gene_symbol": "PRELID1",
  "gene_name": "PRELI domain-containing protein 1, mitochondrial"
}